{
  "term_id": "GO:0005634",
  "term_label": "nucleus",
  "gene_symbol": "NKX2-6",
  "gene_name": "Homeobox protein Nkx-2.6",
  "gene": "UniProtKB:A6NCS4"
}